mesenchymal to epithelial transition involved in metanephros morphogenesis [GO:0003337] (biological process) Definition: A transition where a mesenchymal cell establishes apical/basolateral polarity,forms intercellular adhesive junctions, synthesizes basement membrane components and becomes an epithelial cell that will contribute to the shaping of the metanephros. Sources: GOC:dph, GOC:yaf Also known as: metanephric mesenchyme to epithelial transition Relationships: is a type of epithelial cell differentiation involved in kidney development [GO:0035850]; is a type of GO:0060231; is a type of cell differentiation involved in metanephros development [GO:0072202]; is part of metanephric renal vesicle morphogenesis [GO:0072283] Subtypes: mesenchymal to epithelial transition involved in metanephric renal vesicle formation [GO:0072285] Regulation: regulated by regulation of mesenchymal to epithelial transition involved in metanephros morphogenesis [GO:0003339]; negatively regulated by negative regulation of mesenchymal to epithelial transition involved in metanephros morphogenesis [GO:0003340]; positively regulated by positive regulation of mesenchymal to epithelial transition involved in metanephros morphogenesis [GO:0072108]